imaginal disc-derived genitalia development [GO:0007484] (biological process) Sources: GOC:ai, GOC:sensu Subtypes: imaginal disc-derived male genitalia development [GO:0007485], imaginal disc-derived female genitalia development [GO:0007486] Definition: The process whose specific outcome is the progression of the genitalia over time, from formation as part of the genital disc to the mature structure. An example of this is found in Drosophila melanogaster. Relationships: is a type of genitalia development [GO:0048806]; is part of genital disc development [GO:0035215] Also known as: genital development